{
  "term_id": "UNKNOWN:0002",
  "gene_name": "Zinc finger protein 385C",
  "term_label": "Unknown biological process",
  "gene_symbol": "ZNF385C",
  "gene": "UniProtKB:Q66K41"
}